{
  "term_label": "Unknown cellular component",
  "gene_name": "POU domain, class 3, transcription factor 3",
  "gene": "UniProtKB:P20264",
  "gene_symbol": "POU3F3",
  "term_id": "UNKNOWN:0003"
}